posterior lateral line neuromast hair cell morphogenesis [GO:0035680] (biological process) Relationships: is a type of neuromast hair cell morphogenesis [GO:0035678]; is part of GO:0035677 Definition: The change in form (cell shape and size) that occurs when a posterior lateral line neuromast hair cell progresses from its initial formation to its mature state. A neuromast hair cell is a hair cell that acts as a sensory receptor of the neuromast; it is morphologically polarized as a result of the relative position of the single kinocilium and the clusters of stereocilia on its apical surface. Sources: ISBN:0125296509